copper-nicotianamine transmembrane transporter activity [GO:0051982] (molecular function) Sources: GOC:ai Relationships: is a type of copper chelate transmembrane transporter activity [GO:0051981] Also known as: Cu-NA chelate transporter activity Definition: Enables the transfer of the copper chelate copper-nicotianamine (Cu-NA) from one side of a membrane to the other.